{
  "gene_name": "Metallothionein-1F",
  "gene_symbol": "MT1F",
  "term_label": "metal ion binding",
  "term_id": "GO:0046872",
  "gene": "UniProtKB:P04733"
}